positive regulation of sporangium development [GO:0075311] (biological process) Relationships: is a type of GO:0075261; is a type of regulation of sporangium development [GO:0075310]; positively regulates GO:0043582 Sources: GOC:pamgo_curators Definition: Any process that activates, maintains or increases the frequency, rate or extent of sporangium development, a process that leads to the formation of sporangium, a single-celled or many-celled structure in which spores are produced, as in fungi, algae, mosses, and ferns, gymnosperms, angiosperms. Subtypes: positive regulation of sporangium germination [GO:0075224], positive regulation of oomycete sporangium development [GO:0075323]